{
  "term_id": "GO:0008360",
  "gene_name": "Plexin-D1",
  "gene_symbol": "PLXND1",
  "gene": "UniProtKB:Q9Y4D7",
  "term_label": "regulation of cell shape"
}